{
  "gene_symbol": "VPS16",
  "term_id": "GO:0016197",
  "term_label": "endosomal transport",
  "gene": "UniProtKB:Q9H269",
  "gene_name": "Vacuolar protein sorting-associated protein 16 homolog"
}